{
  "term_label": "Unknown molecular function",
  "term_id": "UNKNOWN:0001",
  "gene_name": "Afadin- and alpha-actinin-binding protein",
  "gene": "UniProtKB:Q9Y2D8",
  "gene_symbol": "SSX2IP"
}